maturation of SSU-rRNA from tetracistronic rRNA transcript (SSU-rRNA, 5.8S rRNA, 2S rRNA, LSU-rRNA) [GO:0000474] (biological process) Sources: GOC:curators Relationships: is a type of maturation of SSU-rRNA [GO:0030490] Definition: Any process involved in the maturation of a precursor Small SubUnit (SSU) ribosomal RNA (rRNA) molecule into a mature SSU-rRNA molecule from the pre-rRNA molecule originally produced as a tetracistronic rRNA transcript that contains the Small Subunit (SSU) rRNA, 5.8 S rRNA, 2S rRNA, and Large Subunit (LSU) in that order from 5' to 3' along the primary transcript.